{
  "gene": "UniProtKB:O60725",
  "gene_symbol": "ICMT",
  "gene_name": "Protein-S-isoprenylcysteine O-methyltransferase",
  "term_label": "endoplasmic reticulum",
  "term_id": "GO:0005783"
}